regulation of protein export from nucleus [GO:0046825] (biological process) Subtypes: negative regulation of protein export from nucleus [GO:0046826], positive regulation of protein export from nucleus [GO:0046827] Definition: Any process that modulates the frequency, rate or extent of the directed movement of proteins from the nucleus to the cytoplasm. Relationships: is a type of GO:0033157; is a type of regulation of nucleocytoplasmic transport [GO:0046822]; regulates GO:0006611 Sources: GOC:bf Also known as: regulation of protein export from cell nucleus, regulation of protein export out of nucleus, regulation of protein transport from nucleus to cytoplasm, regulation of protein-nucleus export